{
  "gene": "UniProtKB:O43847",
  "gene_symbol": "NRDC",
  "gene_name": "Nardilysin",
  "term_label": "proteolysis",
  "term_id": "GO:0006508"
}